{
  "term_id": "UNKNOWN:0002",
  "gene_name": "Trafficking protein particle complex subunit 8",
  "gene_symbol": "TRAPPC8",
  "gene": "UniProtKB:Q9Y2L5",
  "term_label": "Unknown biological process"
}